{
  "term_label": "norepinephrine-epinephrine-mediated vasodilation involved in regulation of systemic arterial blood pressure",
  "gene_name": "Beta-3 adrenergic receptor",
  "gene": "UniProtKB:P13945",
  "gene_symbol": "ADRB3",
  "term_id": "GO:0002025"
}